{
  "gene_symbol": "KPNB1",
  "term_id": "GO:0005634",
  "gene_name": "Importin subunit beta-1",
  "term_label": "nucleus",
  "gene": "UniProtKB:Q14974"
}